(1->6)-beta-D-glucan biosynthetic process [GO:0006078] (biological process) Regulation: regulated by regulation of (1->6)-beta-D-glucan biosynthetic process [GO:0060917] Definition: The chemical reactions and pathways resulting in the formation of (1->6)-beta-D-glucans. Sources: GOC:ai Relationships: is a type of (1->6)-beta-D-glucan metabolic process [GO:0006077]; is_a beta-glucan biosynthetic process [GO:0051274] Also known as: 1,6-beta-glucan anabolism, 1,6-beta-glucan biosynthesis, 1,6-beta-glucan biosynthetic process, 1,6-beta-glucan formation, 1,6-beta-glucan synthesis, beta-1,6 glucan anabolism, beta-1,6 glucan biosynthesis, beta-1,6 glucan biosynthetic process, beta-1,6 glucan formation, beta-1,6 glucan synthesis